{
  "gene_name": "Tumor necrosis factor receptor superfamily member 1B",
  "gene": "UniProtKB:P20333",
  "term_id": "GO:0150079",
  "gene_symbol": "TNFRSF1B",
  "term_label": "negative regulation of neuroinflammatory response"
}